{
  "gene_symbol": "C1QTNF3",
  "term_label": "synapse",
  "gene_name": "Complement C1q tumor necrosis factor-related protein 3",
  "gene": "UniProtKB:Q9BXJ4",
  "term_id": "GO:0045202"
}